{
  "gene": "UniProtKB:Q16385",
  "term_id": "UNKNOWN:0001",
  "term_label": "Unknown molecular function",
  "gene_symbol": "SSX2B",
  "gene_name": "Protein SSX2"
}